{
  "term_id": "UNKNOWN:0002",
  "gene": "UniProtKB:P30046",
  "gene_name": "D-dopachrome decarboxylase",
  "gene_symbol": "DDT",
  "term_label": "Unknown biological process"
}